{
  "gene": "UniProtKB:P01594",
  "gene_symbol": "IGKV1-33",
  "term_label": "immunoglobulin complex",
  "term_id": "GO:0019814",
  "gene_name": "Immunoglobulin kappa variable 1-33"
}